{
  "gene": "UniProtKB:Q8NGC0",
  "gene_name": "Olfactory receptor 5AU1",
  "gene_symbol": "OR5AU1",
  "term_id": "UNKNOWN:0003",
  "term_label": "Unknown cellular component"
}